{
  "gene": "UniProtKB:Q9UPN3",
  "gene_name": "Microtubule-actin cross-linking factor 1, isoforms 1_2_3_4_5",
  "term_label": "regulation of focal adhesion assembly",
  "gene_symbol": "MACF1",
  "term_id": "GO:0051893"
}